{
  "gene": "UniProtKB:Q6P6C2",
  "gene_name": "RNA demethylase ALKBH5",
  "term_id": "GO:0005634",
  "gene_symbol": "ALKBH5",
  "term_label": "nucleus"
}